regulation of myelination [GO:0031641] (biological process) Relationships: is a type of regulation of cellular process [GO:0050794]; is a type of regulation of nervous system development [GO:0051960]; regulates myelination [GO:0042552] Sources: GOC:mah Subtypes: negative regulation of myelination [GO:0031642], positive regulation of myelination [GO:0031643] Definition: Any process that modulates the frequency, rate or extent of the formation of a myelin sheath around nerve axons.